{
  "term_label": "Golgi to plasma membrane transport",
  "gene_name": "Rab GTPase-binding effector protein 1",
  "gene_symbol": "RABEP1",
  "gene": "UniProtKB:Q15276",
  "term_id": "GO:0006893"
}